{
  "gene_symbol": "AQP8",
  "gene_name": "Aquaporin-8",
  "term_label": "plasma membrane",
  "gene": "UniProtKB:O94778",
  "term_id": "GO:0005886"
}